{
  "term_label": "immunoglobulin complex",
  "gene_symbol": "TRAV14DV4",
  "term_id": "GO:0019814",
  "gene": "UniProtKB:A0A0A6YYC5",
  "gene_name": "T cell receptor alpha variable 14_delta variable 4"
}